{
  "gene_name": "Glutamine-rich protein 2",
  "gene_symbol": "QRICH2",
  "term_id": "GO:0036126",
  "term_label": "sperm flagellum",
  "gene": "UniProtKB:Q9H0J4"
}